bisphenol A catabolic process [GO:0043636] (biological process) Definition: The chemical reactions and pathways resulting in the breakdown of bisphenol A, 4,4'-(propane-2,2-diyl)diphenol, a synthetic, aromatic organic compound used as a monomer in the manufacture of polycarbonate plastic and in the manufacture of epoxy resins. Sources: GOC:jl, Wikipedia:Bisphenol_A Also known as: bisphenol-A catabolic process, bisphenol-A catabolism Relationships: is a type of phenol-containing compound catabolic process [GO:0019336]; is_a xenobiotic catabolic process [GO:0042178]